{
  "gene_symbol": "BANK1",
  "term_id": "GO:0005102",
  "term_label": "signaling receptor binding",
  "gene": "UniProtKB:Q8NDB2",
  "gene_name": "B-cell scaffold protein with ankyrin repeats"
}